{
  "gene_symbol": "DNAJB12",
  "term_id": "GO:0005789",
  "gene_name": "DnaJ homolog subfamily B member 12",
  "term_label": "endoplasmic reticulum membrane",
  "gene": "UniProtKB:Q9NXW2"
}